{
  "gene": "UniProtKB:H3BQJ8",
  "term_label": "plasma membrane",
  "gene_name": "Lymphocyte antigen 6L",
  "gene_symbol": "LY6L",
  "term_id": "GO:0005886"
}